{
  "gene": "UniProtKB:P35321",
  "term_id": "GO:0030280",
  "gene_name": "Cornifin-A",
  "term_label": "structural constituent of skin epidermis",
  "gene_symbol": "SPRR1A"
}